{
  "gene": "UniProtKB:P24158",
  "term_label": "proteolysis",
  "term_id": "GO:0006508",
  "gene_symbol": "PRTN3",
  "gene_name": "Myeloblastin"
}